FMN transmembrane transporter activity [GO:0044610] (molecular function) Definition: Enables the directed movement of flavine mononucleotide (FMN) from one side of a membrane to the other. Relationships: is a type of nucleotide transmembrane transporter activity [GO:0015215]; is a type of carbohydrate derivative transmembrane transporter activity [GO:1901505] Also known as: flavine mononucleotide transmembrane transporter activity References: PMID:22185573 Sources: GOC:ans